positive regulation of adult chitin-containing cuticle pigmentation [GO:0048084] (biological process) Definition: Any process that activates or increases the frequency, rate or extent of establishment of the adult pattern of pigmentation in the cuticle of an organism. Also known as: up regulation of adult chitin-containing cuticle pigmentation, up-regulation of adult chitin-containing cuticle pigmentation, upregulation of adult chitin-containing cuticle pigmentation, activation of adult chitin-containing cuticle pigmentation, stimulation of adult chitin-containing cuticle pigmentation Sources: GOC:jid, GOC:mtg_sensu Relationships: is a type of GO:0045801; is a type of positive regulation of cuticle pigmentation [GO:0048081]; is a type of regulation of adult chitin-containing cuticle pigmentation [GO:0048082]; positively regulates adult chitin-containing cuticle pigmentation [GO:0048085]